{
  "gene": "UniProtKB:P04118",
  "gene_symbol": "CLPS",
  "term_label": "Unknown cellular component",
  "gene_name": "Colipase",
  "term_id": "UNKNOWN:0003"
}